{
  "gene": "UniProtKB:Q9P0L9",
  "term_id": "GO:0005509",
  "term_label": "calcium ion binding",
  "gene_name": "Polycystin-2-like protein 1",
  "gene_symbol": "PKD2L1"
}